{
  "gene_symbol": "SMIM3",
  "term_id": "UNKNOWN:0003",
  "gene": "UniProtKB:Q9BZL3",
  "term_label": "Unknown cellular component",
  "gene_name": "Small integral membrane protein 3"
}